{
  "gene": "UniProtKB:Q9H115",
  "gene_symbol": "NAPB",
  "term_id": "GO:0006886",
  "gene_name": "Beta-soluble NSF attachment protein",
  "term_label": "intracellular protein transport"
}